{
  "term_id": "UNKNOWN:0001",
  "gene_name": "Putative glutathione hydrolase light chain 3",
  "gene_symbol": "GGTLC3",
  "term_label": "Unknown molecular function",
  "gene": "UniProtKB:B5MD39"
}